{
  "term_label": "nucleus",
  "gene": "UniProtKB:B2RPK0",
  "gene_symbol": "HMGB1P1",
  "gene_name": "Putative high mobility group protein B1-like 1",
  "term_id": "GO:0005634"
}